{
  "term_label": "Unknown molecular function",
  "term_id": "UNKNOWN:0001",
  "gene": "UniProtKB:Q3SXY7",
  "gene_symbol": "LRIT3",
  "gene_name": "Leucine-rich repeat, immunoglobulin-like domain and transmembrane domain-containing protein 3"
}